viral release via disruption of host peptidoglycan cell wall [GO:0140913] (biological process) Definition: The dissemination of mature viral particles from a host cell, caused by a virus hydrolyzing the peptidoglycan cell wall of the host organism. Peptidoglycans are any of a class of glycoconjugates found in bacterial cell walls. Relationships: is a type of viral release from host cell by cytolysis [GO:0044659] References: PMID:24585055, PMID:26085488, PMID:29495305